deubiquitinase activator activity [GO:0035800] (molecular function) Definition: Binds to and increases the activity of a deubiquitinase. Relationships: is a type of peptidase activator activity [GO:0016504]; positively regulates GO:0101005 Sources: GOC:sart, ISBN:0120793709